{
  "term_id": "GO:0010506",
  "gene_symbol": "ULK2",
  "gene_name": "Serine_threonine-protein kinase ULK2",
  "gene": "UniProtKB:Q8IYT8",
  "term_label": "regulation of autophagy"
}